{
  "term_id": "GO:0043025",
  "gene_symbol": "KCNN2",
  "gene": "UniProtKB:Q9H2S1",
  "gene_name": "Small conductance calcium-activated potassium channel protein 2",
  "term_label": "neuronal cell body"
}